pyridine-containing compound metabolic process [GO:0072524] (biological process) Definition: The chemical reactions and pathways involving a pyridine-containing compound, i.e. any compound that contains pyridine or a formal derivative thereof. Relationships: is_a GO:0008152 Subtypes: nicotinamide metabolic process [GO:0006769], vitamin B6 metabolic process [GO:0042816], nicotinamide nucleotide metabolic process [GO:0046496], quinolinate metabolic process [GO:0046874], GO:0070637, pyridine-containing compound biosynthetic process [GO:0072525], pyridine-containing compound catabolic process [GO:0072526], GO:1901847 Also known as: pyridine and derivative metabolic process, pyridine-containing compound metabolism Sources: GOC:mah